bacteriochlorophyll catabolic process [GO:0030495] (biological process) Sources: GOC:go_curators Definition: The chemical reactions and pathways resulting in the breakdown of bacteriochlorophyll, any of the chlorophylls of photosynthetic bacteria. They differ structurally from the chlorophylls of higher plants. Also known as: bacteriochlorophyll breakdown, bacteriochlorophyll catabolism, bacteriochlorophyll degradation Relationships: is a type of GO:0015996